archaeosine synthase activity [GO:0002948] (molecular function) Definition: Catalysis of the reaction: L-glutamine + 7-cyano-7-carbaguanine15 in tRNA + H2O = L-glutamate + archaeine15 in tRNA. References: PMID:20129918 Sources: RHEA:54084 Also known as: ArcS, glutamine:preQ0-tRNA amidinotransferase Relationships: is a type of transferase activity, transferring nitrogenous groups [GO:0016769]